left lateral basal body pair [GO:0097562] (cellular component) Relationships: is a type of cellular anatomical structure [GO:0110165]; is part of GO:0042995; has part GO:1902671; has part GO:1902675 Note: Due to the asymmetric nature of the Giardia trophozoite, this term is defined spatially as the trophozoite is viewed from the dorsal side, with the two nuclei dorsal to the ventral disc, and the ventral disc toward the anterior. Definition: Set of two basal bodies found in Giardia species (trophozoite stage). It comprises the anterior and ventral basal bodies located to the right of the left nucleus of the trophozoite when viewed dorsally. References: PMID:16607022, PMID:5961344 Sources: GOC:giardia, ISBN:9780124260207